promoter clearance during DNA-templated transcription [GO:0001109] (biological process) Also known as: promoter escape, promoter clearance during DNA-dependent transcription, promoter clearance from bacterial-type RNA polymerase promoter Definition: Any process involved in the transition from the initiation to the elongation phases of transcription by a DNA-dependent RNA polymerase, generally including a conformational change from the initiation conformation to the elongation conformation. Promoter clearance often involves breaking contact with transcription factors involved only in the initiation phase and making contacts with elongation specific factors. References: PMID:15020047, PMID:18280161 Sources: GOC:txnOH Subtypes: RNA polymerase III promoter clearance [GO:0001110], RNA polymerase II promoter clearance [GO:0001111], GO:0001182 Relationships: is a type of RNA biosynthetic process [GO:0032774]; is part of GO:0006351; has part protein-DNA-RNA complex remodeling [GO:0001119]